{
  "term_label": "platelet aggregation",
  "gene": "UniProtKB:Q86UX7",
  "gene_symbol": "FERMT3",
  "term_id": "GO:0070527",
  "gene_name": "Fermitin family homolog 3"
}